{
  "term_id": "GO:0005634",
  "gene": "UniProtKB:Q9Y4X4",
  "gene_symbol": "KLF12",
  "gene_name": "Krueppel-like factor 12",
  "term_label": "nucleus"
}